{
  "term_label": "calcium ion import across plasma membrane",
  "gene_symbol": "TRPV6",
  "gene_name": "Transient receptor potential cation channel subfamily V member 6",
  "gene": "UniProtKB:Q9H1D0",
  "term_id": "GO:0098703"
}